{
  "gene_symbol": "CARTPT",
  "gene": "UniProtKB:Q16568",
  "gene_name": "Cocaine- and amphetamine-regulated transcript protein",
  "term_label": "cellular response to starvation",
  "term_id": "GO:0009267"
}